{
  "gene_name": "BBSome-interacting protein 1",
  "gene_symbol": "BBIP1",
  "term_label": "BBSome",
  "term_id": "GO:0034464",
  "gene": "UniProtKB:A8MTZ0"
}